{
  "term_label": "RNA polymerase II transcription regulatory region sequence-specific DNA binding",
  "gene": "UniProtKB:P81133",
  "gene_symbol": "SIM1",
  "term_id": "GO:0000977",
  "gene_name": "Single-minded homolog 1"
}